steroid 9-alpha-monooxygenase activity [GO:0050292] (molecular function) Sources: RHEA:19557 Definition: Catalysis of the reaction: AH2 + O2 + pregna-4,9(11)-diene-3,20-dione = 9,11alpha-epoxypregn-4-ene-3,20-dione + A + H2O. Also known as: steroid 9a-monooxygenase activity, steroid 9-alpha-hydroxylase activity, steroid 9alpha-hydroxylase activity, steroid 9alpha-monooxygenase activity, steroid,hydrogen-donor:oxygen oxidoreductase (9-epoxidizing) Relationships: is a type of steroid hydroxylase activity [GO:0008395]; is a type of oxidoreductase activity, acting on paired donors, with incorporation or reduction of molecular oxygen [GO:0016705]